water channel activity [GO:0015250] (molecular function) Definition: Enables the energy-independent facilitated diffusion of water through a transmembrane aqueous pore or channel. Regulation: regulated by regulation of water channel activity [GO:1902427] Sources: GOC:mtg_transport, ISBN:0815340729 Relationships: is a type of water transmembrane transporter activity [GO:0005372]; is a type of channel activity [GO:0015267] Also known as: aquaporin